D-allose transmembrane transport [GO:0015754] (biological process) Definition: The process in which D-allose is transported across a lipid bilayer, from one side of a membrane to the other. Allose is an aldohexose similar to glucose, differing only in the configuration of the hydroxyl group of C-3. Also known as: allose transmembrane transport, allose transport Sources: GOC:ai Relationships: is a type of GO:0008645